TFIIB-class transcription factor binding [GO:0001093] (molecular function) Definition: Binding to a general RNA polymerase II transcription factor of the TFIIB class, one of the factors involved in formation of the preinitiation complex (PIC) by RNA polymerase II. Relationships: is a type of RNA polymerase II general transcription initiation factor binding [GO:0001091] References: PMID:16858867 Sources: GOC:krc